{
  "term_id": "GO:0008307",
  "term_label": "structural constituent of muscle",
  "gene": "UniProtKB:Q16527",
  "gene_symbol": "CSRP2",
  "gene_name": "Cysteine and glycine-rich protein 2"
}